{
  "gene": "UniProtKB:P56270",
  "gene_symbol": "MAZ",
  "gene_name": "Myc-associated zinc finger protein",
  "term_label": "RNA polymerase II cis-regulatory region sequence-specific DNA binding",
  "term_id": "GO:0000978"
}